{
  "gene_name": "Zinc finger protein 583",
  "term_id": "GO:0006357",
  "gene": "UniProtKB:Q96ND8",
  "term_label": "regulation of transcription by RNA polymerase II",
  "gene_symbol": "ZNF583"
}